{
  "gene": "UniProtKB:Q13367",
  "gene_symbol": "AP3B2",
  "gene_name": "AP-3 complex subunit beta-2",
  "term_id": "UNKNOWN:0001",
  "term_label": "Unknown molecular function"
}